negative regulation of neurotransmitter secretion [GO:0046929] (biological process) Definition: Any process that stops, prevents, or reduces the frequency, rate or extent of the regulated release of a neurotransmitter. Sources: GOC:ai Also known as: down regulation of neurotransmitter secretion, down-regulation of neurotransmitter secretion, downregulation of neurotransmitter secretion, conotoxin activity, inhibition of neurotransmitter secretion Relationships: is a type of regulation of neurotransmitter secretion [GO:0046928]; is a type of negative regulation of neurotransmitter transport [GO:0051589]; is a type of GO:1903531; RO_0002212 neurotransmitter secretion [GO:0007269] Subtypes: negative regulation of acetylcholine secretion, neurotransmission [GO:0014058], negative regulation of glutamate secretion, neurotransmission [GO:1903295], GO:1904049, negative regulation of substance P secretion, neurotransmission [GO:1904495], negative regulation of glycine secretion, neurotransmission [GO:1904625]